male gamete generation [GO:0048232] (biological process) Relationships: is a type of GO:0007276 Sources: GOC:dph, GOC:jid Subtypes: spermatogenesis [GO:0007283] Definition: Generation of the male gamete; specialised haploid cells produced by meiosis and along with a female gamete takes part in sexual reproduction.